{
  "term_id": "UNKNOWN:0002",
  "gene_symbol": "VSTM2A",
  "term_label": "Unknown biological process",
  "gene": "UniProtKB:Q8TAG5",
  "gene_name": "V-set and transmembrane domain-containing protein 2A"
}